{
  "gene": "UniProtKB:Q5XG92",
  "term_label": "Unknown cellular component",
  "gene_name": "Carboxylesterase 4A",
  "term_id": "UNKNOWN:0003",
  "gene_symbol": "CES4A"
}